{
  "gene": "UniProtKB:Q14449",
  "term_id": "GO:0046627",
  "gene_name": "Growth factor receptor-bound protein 14",
  "gene_symbol": "GRB14",
  "term_label": "negative regulation of insulin receptor signaling pathway"
}